DNA protection [GO:0042262] (biological process) Definition: Any process in which DNA is protected from damage by, for example, oxidative stress. Sources: GOC:jl Relationships: is a type of DNA metabolic process [GO:0006259]; is a type of GO:0033554